{
  "term_id": "GO:0006936",
  "gene_symbol": "MYH1",
  "gene_name": "Myosin-1",
  "gene": "UniProtKB:P12882",
  "term_label": "muscle contraction"
}